{
  "gene_name": "Neurogenin-2",
  "term_label": "nucleus",
  "term_id": "GO:0005634",
  "gene": "UniProtKB:Q9H2A3",
  "gene_symbol": "NEUROG2"
}